{
  "term_label": "establishment of sister chromatid cohesion",
  "term_id": "GO:0034085",
  "gene_symbol": "DDX11",
  "gene_name": "ATP-dependent DNA helicase DDX11",
  "gene": "UniProtKB:Q96FC9"
}